{
  "gene_symbol": "CCNG1",
  "term_label": "nucleus",
  "gene": "UniProtKB:P51959",
  "gene_name": "Cyclin-G1",
  "term_id": "GO:0005634"
}